{
  "gene_symbol": "ADCK5",
  "gene": "UniProtKB:Q3MIX3",
  "term_label": "Unknown molecular function",
  "gene_name": "Uncharacterized aarF domain-containing protein kinase 5",
  "term_id": "UNKNOWN:0001"
}